endolysosomal toll-like receptor signaling pathway [GO:0140894] (biological process) Subtypes: toll-like receptor 3 signaling pathway [GO:0034138], toll-like receptor 7 signaling pathway [GO:0034154], toll-like receptor 8 signaling pathway [GO:0034158], toll-like receptor 9 signaling pathway [GO:0034162], GO:0034170, toll-like receptor 12 signaling pathway [GO:0034174], toll-like receptor 13 signaling pathway [GO:0034178] References: PMID:29679565 Relationships: is a type of cytoplasmic pattern recognition receptor signaling pathway [GO:0002753] Also known as: endolysosomal pattern recognition receptor signaling pathway Definition: The series of molecular signals initiated by a ligand binding to an endolysosomal pattern recognition receptor (PRR) of the toll-like family. PRRs bind pathogen-associated molecular pattern (PAMPs), structures conserved among microbial species.